{
  "term_label": "GTPase activity",
  "gene_name": "GTPase KRas",
  "gene_symbol": "KRAS",
  "term_id": "GO:0003924",
  "gene": "UniProtKB:P01116"
}